{
  "gene_symbol": "UBL5",
  "gene_name": "Ubiquitin-like protein 5",
  "term_id": "GO:0031386",
  "gene": "UniProtKB:Q9BZL1",
  "term_label": "protein tag activity"
}